{
  "term_label": "Unknown molecular function",
  "gene_symbol": "SNF8",
  "gene_name": "Vacuolar-sorting protein SNF8",
  "term_id": "UNKNOWN:0001",
  "gene": "UniProtKB:Q96H20"
}